ventricular septum intermedium morphogenesis [GO:0003288] (biological process) Sources: GOC:mtg_heart Definition: The developmental process in which a ventricular septum intermedium is generated and organized. Relationships: is a type of ventricular septum morphogenesis [GO:0060412]